unidirectional conjugation [GO:0009291] (biological process) Relationships: is a type of GO:0009292 Subtypes: pheromone-induced unidirectional conjugation [GO:0000762] Sources: Wikipedia:Bacterial_conjugation Also known as: bacterial conjugation Note: Unidirectional conjugation is not a type of not sexual reproduction, since no exchange of gamete occurs and no generation of a new organism: instead an existing organism is transformed. Definition: The process of unidirectional (polarized) transfer of genetic information involving direct cellular contact between a donor and recipient cell; the contact is followed by the formation of a cellular bridge that physically connects the cells. Some or all of the chromosome(s) of the donor cell is transferred into the recipient cell.